replication fork barrier binding [GO:0031634] (molecular function) Definition: Binding to replication fork barriers, sites that inhibit the progress of replication forks. Relationships: is a type of GO:1990837 Subtypes: rDNA spacer replication fork barrier binding [GO:0043110], mating type region replication fork barrier binding [GO:1990943] Sources: GOC:mah